{
  "term_id": "UNKNOWN:0003",
  "gene_symbol": "VWA5B2",
  "gene_name": "von Willebrand factor A domain-containing protein 5B2",
  "term_label": "Unknown cellular component",
  "gene": "UniProtKB:Q8N398"
}